{
  "gene_symbol": "ATOH8",
  "gene_name": "Transcription factor ATOH8",
  "gene": "UniProtKB:Q96SQ7",
  "term_label": "DNA-binding transcription factor activity",
  "term_id": "GO:0003700"
}